dynein light chain binding [GO:0045503] (molecular function) Relationships: is a type of protein binding [GO:0005515] Sources: GOC:bf Definition: Binding to a light chain of the dynein complex.